regulation protein catabolic process at synapse [GO:0140250] (biological process) Note: Note that this term was created for the SynGO project, and will be obsoleted when the SynGO annotations are made in Noctua. Subtypes: regulation of protein catabolic process at synapse, modulating synaptic transmission [GO:0099574], regulation protein catabolic process at presynapse [GO:0140251], regulation protein catabolic process at postsynapse [GO:0140252] Definition: Any process that modulates the frequency, rate or extent of the chemical reactions and pathways resulting in the breakdown of a protein at the synapse. References: PMID:23083742 Relationships: is a type of regulation of catabolic process [GO:0009894]; occurs in synapse [GO:0045202]